cellular response to paraquat [GO:0072756] (biological process) Definition: Any process that results in a change in state or activity of a cell (in terms of movement, secretion, enzyme production, gene expression, etc.) as a result of a paraquat stimulus. Relationships: is a type of cellular response to chemical stimulus [GO:0070887]; is a type of GO:1901562 Sources: GOC:mah